protein kinase regulator activity [GO:0019887] (molecular function) Relationships: is a type of kinase regulator activity [GO:0019207]; has part GO:0019901; regulates protein kinase activity [GO:0004672] Definition: Modulates the activity of a protein kinase, an enzyme which phosphorylates a protein. Subtypes: protein kinase inhibitor activity [GO:0004860], GO:0008603, phosphorylase kinase regulator activity [GO:0008607], calcium-dependent protein kinase regulator activity [GO:0010858], cyclin-dependent protein kinase regulator activity [GO:0019914], GO:0030295, eukaryotic elongation factor-2 kinase regulator activity [GO:0042556] Sources: GOC:ai